{
  "term_id": "GO:0005615",
  "gene_symbol": "MYOC",
  "gene_name": "Myocilin",
  "term_label": "extracellular space",
  "gene": "UniProtKB:Q99972"
}